{
  "term_label": "spindle",
  "term_id": "GO:0005819",
  "gene": "UniProtKB:A8MVW5",
  "gene_symbol": "HEPACAM2",
  "gene_name": "HEPACAM family member 2"
}